{
  "gene": "UniProtKB:Q7Z7F0",
  "term_label": "RNA binding",
  "term_id": "GO:0003723",
  "gene_name": "KH homology domain-containing protein 4",
  "gene_symbol": "KHDC4"
}